{
  "gene_name": "Rho-related GTP-binding protein RhoG",
  "term_label": "regulation of cell shape",
  "gene_symbol": "RHOG",
  "gene": "UniProtKB:P84095",
  "term_id": "GO:0008360"
}